ER ubiquitin ligase complex [GO:0000835] (cellular component) Definition: A ubiquitin ligase complex found in the ER. Sources: GOC:elh Relationships: is a type of cytoplasmic ubiquitin ligase complex [GO:0000153]; is a type of membrane protein complex [GO:0098796]; is a type of endoplasmic reticulum protein-containing complex [GO:0140534]; is part of endoplasmic reticulum membrane [GO:0005789] Subtypes: Hrd1p ubiquitin ligase complex [GO:0000836], Doa10p ubiquitin ligase complex [GO:0000837], CUE1-UBC7 ubiquitin-conjugating enzyme complex [GO:1990389]